{
  "gene": "UniProtKB:O00585",
  "gene_symbol": "CCL21",
  "term_label": "extracellular space",
  "term_id": "GO:0005615",
  "gene_name": "C-C motif chemokine 21"
}